{
  "gene_name": "UBX domain-containing protein 1",
  "term_id": "GO:0005634",
  "term_label": "nucleus",
  "gene": "UniProtKB:Q04323",
  "gene_symbol": "UBXN1"
}